{
  "term_label": "membrane",
  "gene_symbol": "A0A286YEU6",
  "gene": "UniProtKB:A0A286YEU6",
  "term_id": "GO:0016020",
  "gene_name": "Olfactory receptor family 1 subfamily R member 1 pseudogene"
}